{
  "gene_name": "RB1-inducible coiled-coil protein 1",
  "gene_symbol": "RB1CC1",
  "term_label": "phagophore assembly site membrane",
  "term_id": "GO:0034045",
  "gene": "UniProtKB:Q8TDY2"
}